{
  "gene_name": "Septin-14",
  "gene_symbol": "SEPTIN14",
  "gene": "UniProtKB:Q6ZU15",
  "term_label": "GTPase activity",
  "term_id": "GO:0003924"
}